{
  "gene_symbol": "KIAA1191",
  "gene_name": "Putative monooxygenase p33MONOX",
  "term_label": "cytoplasm",
  "gene": "UniProtKB:Q96A73",
  "term_id": "GO:0005737"
}